{
  "gene": "UniProtKB:P16298",
  "gene_symbol": "PPP3CB",
  "term_label": "calcineurin-mediated signaling",
  "gene_name": "Serine_threonine-protein phosphatase 2B catalytic subunit beta isoform",
  "term_id": "GO:0097720"
}